glucagon receptor binding [GO:0031769] (molecular function) Also known as: glucagon receptor ligand Sources: GOC:mah, GOC:nln Definition: Binding to a glucagon receptor. Relationships: is a type of G protein-coupled receptor binding [GO:0001664]